{
  "gene_symbol": "IBTK",
  "term_label": "protein tyrosine kinase inhibitor activity",
  "gene": "UniProtKB:Q9P2D0",
  "gene_name": "Inhibitor of Bruton tyrosine kinase",
  "term_id": "GO:0030292"
}